von-Willerbrand-factor-A-domain-rich collagen trimer [GO:0140158] (cellular component) Subtypes: collagen type VI trimer [GO:0005589], collagen type VII trimer [GO:0005590], collagen type XXVIII trimer [GO:1990326] Relationships: is a type of GO:0005581 References: PMID:21421911 Definition: A family of collagens containing multiple von Willebrand factor A (vWA) domains.